positive regulation of calcium ion transport [GO:0051928] (biological process) Definition: Any process that activates or increases the frequency, rate or extent of the directed movement of calcium ions into, out of or within a cell, or between cells, by means of some agent such as a transporter or pore. Also known as: positive regulation of calcium transport, up regulation of calcium ion transport, up-regulation of calcium ion transport, upregulation of calcium ion transport, activation of calcium ion transport, stimulation of calcium ion transport Sources: GOC:ai Relationships: is a type of positive regulation of monoatomic ion transport [GO:0043270]; is a type of regulation of calcium ion transport [GO:0051924]; positively regulates calcium ion transport [GO:0006816] Subtypes: positive regulation of calcium ion import [GO:0090280], GO:0106129, positive regulation of calcium ion import into sarcoplasmic reticulum [GO:1902082], positive regulation of calcium ion transmembrane transport [GO:1904427]